{
  "gene": "UniProtKB:P61956",
  "term_label": "protein tag activity",
  "gene_name": "Small ubiquitin-related modifier 2",
  "gene_symbol": "SUMO2",
  "term_id": "GO:0031386"
}